COPI coating of Golgi vesicle, cis-Golgi to rough ER [GO:0010788] (BP) Sources: GOC:dph, GOC:tb Relationships: is_a COPI coating of Golgi vesicle [GO:0048205]; is part of vesicle targeting, cis-Golgi to rough endoplasmic reticulum [GO:0048206] Definition: The addition of COPI proteins and adaptor proteins to Golgi membranes during the formation of cis-Golgi to rough ER transport vesicles, forming a vesicle coat.